response to borneol [GO:1905230] (BP) Definition: Any process that results in a change in state or activity of a cell or an organism (in terms of movement, secretion, enzyme production, gene expression, etc.) as a result of a borneol stimulus. Subtypes: cellular response to borneol [GO:1905231] References: PMID:26593909 Sources: GOC:TermGenie, GO_REF:0000071 Relationships: is a type of response to lipid [GO:0033993]